{
  "term_id": "UNKNOWN:0001",
  "gene_name": "Selenoprotein P",
  "term_label": "Unknown molecular function",
  "gene": "UniProtKB:P49908",
  "gene_symbol": "SELENOP"
}